{
  "term_id": "UNKNOWN:0001",
  "term_label": "Unknown molecular function",
  "gene_name": "Phytanoyl-CoA dioxygenase domain-containing protein 1",
  "gene": "UniProtKB:Q5SRE7",
  "gene_symbol": "PHYHD1"
}